{
  "gene": "UniProtKB:A6NIJ5",
  "term_id": "UNKNOWN:0002",
  "gene_symbol": "FAM90A20P",
  "gene_name": "Putative protein FAM90A20P",
  "term_label": "Unknown biological process"
}